{
  "term_label": "olfactory receptor activity",
  "gene_name": "Olfactory receptor 4D6",
  "term_id": "GO:0004984",
  "gene_symbol": "OR4D6",
  "gene": "UniProtKB:Q8NGJ1"
}